cellular response to cocaine [GO:0071314] (biological process) Definition: Any process that results in a change in state or activity of a cell (in terms of movement, secretion, enzyme production, gene expression, etc.) as a result of a cocaine stimulus. Cocaine is a crystalline alkaloid obtained from the leaves of the coca plant. Relationships: is a type of response to cocaine [GO:0042220]; is a type of cellular response to alkaloid [GO:0071312]; is a type of cellular response to oxygen-containing compound [GO:1901701] Sources: GOC:mah